{
  "gene_name": "Rab11 family-interacting protein 5",
  "gene": "UniProtKB:Q9BXF6",
  "gene_symbol": "RAB11FIP5",
  "term_id": "GO:0005769",
  "term_label": "early endosome"
}